{
  "gene_symbol": "CSK",
  "gene_name": "Tyrosine-protein kinase CSK",
  "term_id": "GO:0005886",
  "gene": "UniProtKB:P41240",
  "term_label": "plasma membrane"
}